{
  "term_id": "UNKNOWN:0003",
  "gene_symbol": "FOXE1",
  "term_label": "Unknown cellular component",
  "gene_name": "Forkhead box protein E1",
  "gene": "UniProtKB:O00358"
}